{
  "gene_name": "Frizzled-9",
  "term_id": "GO:0017147",
  "gene": "UniProtKB:O00144",
  "term_label": "Wnt-protein binding",
  "gene_symbol": "FZD9"
}